{
  "gene": "UniProtKB:Q04743",
  "gene_name": "Homeobox protein EMX2",
  "term_label": "central nervous system development",
  "term_id": "GO:0007417",
  "gene_symbol": "EMX2"
}